{
  "gene": "UniProtKB:P09629",
  "gene_symbol": "HOXB7",
  "gene_name": "Homeobox protein Hox-B7",
  "term_label": "nucleus",
  "term_id": "GO:0005634"
}